{
  "term_id": "GO:0045087",
  "gene_name": "Transcription factor RelB",
  "term_label": "innate immune response",
  "gene_symbol": "RELB",
  "gene": "UniProtKB:Q01201"
}